{
  "term_label": "chloride transport",
  "gene_symbol": "CLIC2",
  "term_id": "GO:0006821",
  "gene_name": "Chloride intracellular channel protein 2",
  "gene": "UniProtKB:O15247"
}